{
  "gene_name": "Uncharacterized protein",
  "gene": "UniProtKB:A0A1W2PNU3",
  "term_label": "Unknown biological process",
  "gene_symbol": "LOC122455342",
  "term_id": "UNKNOWN:0002"
}